{
  "gene": "UniProtKB:P24522",
  "gene_symbol": "GADD45A",
  "term_label": "nucleus",
  "gene_name": "Growth arrest and DNA damage-inducible protein GADD45 alpha",
  "term_id": "GO:0005634"
}